{
  "term_id": "GO:0008277",
  "gene_symbol": "RGS12",
  "gene_name": "Regulator of G-protein signaling 12",
  "term_label": "regulation of G protein-coupled receptor signaling pathway",
  "gene": "UniProtKB:O14924"
}